{
  "gene": "UniProtKB:Q14188",
  "gene_name": "Transcription factor Dp-2",
  "term_label": "nucleus",
  "term_id": "GO:0005634",
  "gene_symbol": "TFDP2"
}